B cell receptor internalization [GO:0036300] (biological process) Subtypes: positive regulation of toll-like receptor 9 signaling pathway by B cell receptor internalization [GO:1901245] Sources: GOC:add, GOC:amm Relationships: is a type of receptor internalization [GO:0031623] Definition: A receptor-mediated endocytosis process that results in the movement of a B cell receptor from the plasma membrane to the inside of the cell. Also known as: BCR endocytosis, BCR receptor internalization, B cell receptor uptake of antigen